{
  "gene": "UniProtKB:O60682",
  "gene_name": "Musculin",
  "gene_symbol": "MSC",
  "term_label": "Unknown cellular component",
  "term_id": "UNKNOWN:0003"
}